regulation of lymphatic vessel size [GO:1990186] (biological process) Subtypes: collecting lymphatic vessel constriction [GO:1990192] Also known as: regulation of collecting lymphatic vessel size Relationships: is a type of GO:0090066; is a type of lymphatic vascular process in circulatory system [GO:1990183] Definition: Any process that modulates the size of lymphatic vessels. References: PMID:23897233